NAD-dependent protein de-2-hydroxyisobutyrylase activity [GO:0160013] (molecular function) Definition: Catalysis of the reaction: H2O + N6-(2-hydroxyisobutanoyl)-L-lysyl-[protein] + NAD+ = 2''-O-(2-hydroxyisobutanoyl)-ADP-D-ribose + L-lysyl-[protein] + nicotinamide. Relationships: is a type of acyltransferase activity, transferring groups other than amino-acyl groups [GO:0016747] References: PMID:31328167